{
  "gene_name": "UBX domain-containing protein 2A",
  "term_id": "GO:0000045",
  "gene": "UniProtKB:P68543",
  "gene_symbol": "UBXN2A",
  "term_label": "autophagosome assembly"
}